{
  "term_label": "cell-cell adhesion",
  "term_id": "GO:0098609",
  "gene": "UniProtKB:Q93052",
  "gene_name": "Lipoma-preferred partner",
  "gene_symbol": "LPP"
}